{
  "gene_symbol": "KDR",
  "term_id": "GO:0019838",
  "gene": "UniProtKB:P35968",
  "term_label": "growth factor binding",
  "gene_name": "Vascular endothelial growth factor receptor 2"
}